{
  "term_id": "GO:0016358",
  "gene_name": "Microtubule-associated protein 1A",
  "term_label": "dendrite development",
  "gene": "UniProtKB:P78559",
  "gene_symbol": "MAP1A"
}